{
  "gene_symbol": "GABARAPL2",
  "gene": "UniProtKB:P60520",
  "term_id": "GO:0031625",
  "gene_name": "Gamma-aminobutyric acid receptor-associated protein-like 2",
  "term_label": "ubiquitin protein ligase binding"
}